{
  "gene": "UniProtKB:P22310",
  "term_label": "flavone metabolic process",
  "gene_symbol": "UGT1A4",
  "term_id": "GO:0051552",
  "gene_name": "UDP-glucuronosyltransferase 1A4"
}